{
  "term_label": "receptor recycling",
  "gene_name": "Pleckstrin homology domain-containing family A member 3",
  "gene": "UniProtKB:Q9HB20",
  "gene_symbol": "PLEKHA3",
  "term_id": "GO:0001881"
}